limbic system development [GO:0021761] (biological process) Sources: GOC:cls, GOC:dgh, GOC:dph, GOC:jid, GO_REF:0000021 Definition: The progression of the limbic system over time from its initial formation until its mature state. The limbic system is a collection of structures in the brain involved in emotion, motivation and emotional aspects of memory. Relationships: is a type of system development [GO:0048731]; is part of forebrain development [GO:0030900]